{
  "gene": "UniProtKB:Q9Y586",
  "gene_name": "Protein mab-21-like 2",
  "gene_symbol": "MAB21L2",
  "term_id": "UNKNOWN:0001",
  "term_label": "Unknown molecular function"
}